{
  "gene_name": "T cell receptor beta variable 11-3",
  "gene_symbol": "TRBV11-3",
  "term_label": "Unknown molecular function",
  "term_id": "UNKNOWN:0001",
  "gene": "UniProtKB:A0A5A6"
}